{
  "gene": "UniProtKB:P17677",
  "term_id": "GO:0001786",
  "gene_name": "Neuromodulin",
  "term_label": "phosphatidylserine binding",
  "gene_symbol": "GAP43"
}